response to acetate [GO:0010034] (biological process) Sources: GOC:sm Regulation: regulated by regulation of response to acetate [GO:1901457]; negatively regulated by negative regulation of response to acetate [GO:1901458]; positively regulated by GO:1901459 Subtypes: cellular response to acetate [GO:0071311] Relationships: is_a GO:1901700 Definition: Any process that results in a change in state or activity of a cell or an organism (in terms of movement, secretion, enzyme production, gene expression, etc.) as a result of an acetate stimulus.